mitochondrial envelope [GO:0005740] (cellular component) Relationships: is a type of organelle envelope [GO:0031967]; BFO_0000050 mitochondrion [GO:0005739] Sources: GOC:ai, GOC:pz Definition: The double lipid bilayer enclosing the mitochondrion and separating its contents from the cell cytoplasm; includes the intermembrane space.